{
  "term_label": "plasma membrane",
  "gene": "UniProtKB:Q96Q06",
  "term_id": "GO:0005886",
  "gene_symbol": "PLIN4",
  "gene_name": "Perilipin-4"
}